{
  "gene": "UniProtKB:Q5HYC2",
  "gene_name": "Uncharacterized protein KIAA2026",
  "gene_symbol": "KIAA2026",
  "term_label": "Unknown cellular component",
  "term_id": "UNKNOWN:0003"
}